{
  "gene_symbol": "FUOM",
  "gene_name": "Fucose mutarotase",
  "term_label": "fucose metabolic process",
  "gene": "UniProtKB:A2VDF0",
  "term_id": "GO:0006004"
}